cytosine binding [GO:0002056] (molecular function) Relationships: is a type of pyrimidine nucleobase binding [GO:0002061] Definition: Binding to cytosine. Sources: GOC:hjd, GOC:vw